{
  "term_id": "UNKNOWN:0003",
  "gene_name": "Casein kinase II subunit alpha'-interacting protein",
  "term_label": "Unknown cellular component",
  "gene_symbol": "CSNKA2IP",
  "gene": "UniProtKB:A0A1B0GTH6"
}